{
  "term_label": "tubulin complex assembly",
  "term_id": "GO:0007021",
  "gene_symbol": "TBCC",
  "gene": "UniProtKB:Q15814",
  "gene_name": "Tubulin-specific chaperone C"
}